{
  "term_label": "Unknown cellular component",
  "gene_symbol": "C11orf42",
  "term_id": "UNKNOWN:0003",
  "gene_name": "Uncharacterized protein C11orf42",
  "gene": "UniProtKB:Q8N5U0"
}